{
  "gene_name": "Cytosolic 10-formyltetrahydrofolate dehydrogenase",
  "term_id": "GO:0004029",
  "term_label": "aldehyde dehydrogenase (NAD+) activity",
  "gene": "UniProtKB:O75891",
  "gene_symbol": "ALDH1L1"
}